cellular response to glucose stimulus [GO:0071333] (biological process) Sources: GOC:mah Definition: Any process that results in a change in state or activity of a cell (in terms of movement, secretion, enzyme production, gene expression, etc.) as a result of a glucose stimulus. Relationships: is a type of intracellular glucose homeostasis [GO:0001678]; is a type of response to glucose [GO:0009749]; is a type of GO:0071331